{
  "gene": "UniProtKB:O75558",
  "term_label": "SNARE binding",
  "gene_symbol": "STX11",
  "term_id": "GO:0000149",
  "gene_name": "Syntaxin-11"
}